{
  "term_label": "Unknown molecular function",
  "term_id": "UNKNOWN:0001",
  "gene_symbol": "SLCO6A1",
  "gene_name": "Solute carrier organic anion transporter family member 6A1",
  "gene": "UniProtKB:Q86UG4"
}